{
  "gene_name": "Carbohydrate sulfotransferase 15",
  "gene_symbol": "CHST15",
  "term_label": "N-acetylgalactosamine 4-sulfate 6-O-sulfotransferase activity",
  "term_id": "GO:0050659",
  "gene": "UniProtKB:Q7LFX5"
}